{
  "term_label": "glycoprotein-fucosylgalactoside alpha-N-acetylgalactosaminyltransferase activity",
  "gene": "UniProtKB:P16442",
  "gene_symbol": "ABO",
  "term_id": "GO:0004380",
  "gene_name": "Histo-blood group ABO system transferase"
}